{
  "term_id": "GO:0043005",
  "gene": "UniProtKB:Q9UPX0",
  "term_label": "neuron projection",
  "gene_symbol": "IGSF9B",
  "gene_name": "Protein turtle homolog B"
}